regulation of protein linear polyubiquitination [GO:1902528] (biological process) Also known as: regulation of M1 linkage References: PMID:21931591 Sources: GOC:TermGenie Relationships: is a type of regulation of protein polyubiquitination [GO:1902914]; regulates protein linear polyubiquitination [GO:0097039] Subtypes: negative regulation of protein linear polyubiquitination [GO:1902529], GO:1902530 Definition: Any process that modulates the frequency, rate or extent of protein linear polyubiquitination.